{
  "gene": "UniProtKB:P01009",
  "term_id": "UNKNOWN:0002",
  "gene_symbol": "SERPINA1",
  "gene_name": "Alpha-1-antitrypsin",
  "term_label": "Unknown biological process"
}